{
  "gene_symbol": "HIPK2",
  "gene": "UniProtKB:Q9H2X6",
  "term_id": "GO:0004713",
  "gene_name": "Homeodomain-interacting protein kinase 2",
  "term_label": "protein tyrosine kinase activity"
}